{
  "gene_symbol": "LIPE",
  "term_id": "GO:0004771",
  "term_label": "sterol ester esterase activity",
  "gene_name": "Hormone-sensitive lipase",
  "gene": "UniProtKB:Q05469"
}